{
  "gene_symbol": "MVK",
  "gene_name": "Mevalonate kinase",
  "term_id": "GO:0005829",
  "gene": "UniProtKB:Q03426",
  "term_label": "cytosol"
}